{
  "term_id": "GO:0006511",
  "term_label": "ubiquitin-dependent protein catabolic process",
  "gene_name": "E3 ubiquitin-protein ligase RNF185",
  "gene": "UniProtKB:Q96GF1",
  "gene_symbol": "RNF185"
}